regulation of calcium-dependent cell-cell adhesion [GO:0046586] (biological process) Sources: GOC:ai Relationships: is a type of GO:0022407; regulates calcium-dependent cell-cell adhesion [GO:0016339] Definition: Any process that modulates the frequency, rate or extent of the attachment of one cell to another cell via adhesion molecules that require the presence of calcium for the interaction. Subtypes: GO:0046587, GO:0046588